{
  "gene": "UniProtKB:P49914",
  "gene_name": "5-formyltetrahydrofolate cyclo-ligase",
  "gene_symbol": "MTHFS",
  "term_id": "GO:0009396",
  "term_label": "folic acid-containing compound biosynthetic process"
}